glycogen synthase activity, transferring glucose-1-phosphate [GO:0061547] (MF) References: PMID:21356517 Sources: GOC:dph Relationships: is_a GO:0016772 Definition: Catalysis of the reaction: UDP-glucose + (1,4)-alpha-D-glucosyl(n) = UMP + (1,4)-alpha-D-glucosyl(n)-glucose-1-phosphate.